{
  "term_id": "GO:0005886",
  "gene_name": "Semaphorin-4D",
  "gene_symbol": "SEMA4D",
  "gene": "UniProtKB:Q92854",
  "term_label": "plasma membrane"
}